stamen development [GO:0048443] (biological process) Definition: The process whose specific outcome is the progression of the stamen over time, from its formation to the mature structure. Sources: GOC:go_curators Relationships: is a type of floral organ development [GO:0048437]; is a type of phyllome development [GO:0048827]; is part of GO:0048466